{
  "gene_name": "Lactosylceramide 1,3-N-acetyl-beta-D-glucosaminyltransferase",
  "gene": "UniProtKB:Q9BYG0",
  "term_label": "Unknown biological process",
  "term_id": "UNKNOWN:0002",
  "gene_symbol": "B3GNT5"
}